{
  "gene_name": "Carnitine O-palmitoyltransferase 1, liver isoform",
  "gene_symbol": "CPT1A",
  "term_label": "fatty acid metabolic process",
  "term_id": "GO:0006631",
  "gene": "UniProtKB:P50416"
}